{
  "gene_name": "Calmodulin-1",
  "term_label": "detection of calcium ion",
  "gene_symbol": "CALM1",
  "term_id": "GO:0005513",
  "gene": "UniProtKB:P0DP23"
}